lens placode formation [GO:0001743] (biological process) Also known as: optic placode formation Subtypes: GO:0046619 Definition: The initial developmental process that will lead to the formation of an eye. Relationships: is a type of ectodermal placode formation [GO:0060788]; is part of embryonic morphogenesis [GO:0048598] Sources: GOC:dph